{
  "gene": "UniProtKB:Q16540",
  "term_id": "GO:0005762",
  "gene_symbol": "MRPL23",
  "gene_name": "Large ribosomal subunit protein uL23m",
  "term_label": "mitochondrial large ribosomal subunit"
}